regulation of kidney size [GO:0035564] (biological process) Subtypes: GO:0035565, GO:0035566 Relationships: is_a regulation of anatomical structure size [GO:0090066]; is part of kidney morphogenesis [GO:0060993] Definition: Any process that modulates the size of a kidney. Sources: GOC:bf